glomerular filtration [GO:0003094] (biological process) Definition: The process in which plasma is filtered through the glomerular membrane which consists of capillary endothelial cells, the basement membrane, and epithelial cells. The glomerular filtrate is the same as plasma except it has no significant amount of protein. Sources: GOC:mtg_cardio, GOC:sart, ISBN:0721643949 Regulation: regulated by regulation of glomerular filtration [GO:0003093]; positively regulated by positive regulation of glomerular filtration [GO:0003104]; negatively regulated by negative regulation of glomerular filtration [GO:0003105] Relationships: is a type of GO:0097205